{
  "gene_symbol": "ABHD14A",
  "term_id": "UNKNOWN:0001",
  "gene": "UniProtKB:Q9BUJ0",
  "term_label": "Unknown molecular function",
  "gene_name": "Protein ABHD14A"
}